mitosome [GO:0032047] (cellular component) Relationships: is a type of intracellular membrane-bounded organelle [GO:0043231]; is part of GO:0005737 Note: In Giardia species, mitosomes are sometimes present between the two nuclei. Also known as: crypton References: PMID:10361303, PMID:14614504, PMID:24316280 Sources: GOC:giardia Definition: A double-membrane-bounded organelle that functions in iron-sulfur protein maturation; evolutionarily derived from mitochondria. The mitosome has been detected only in anaerobic or microaerophilic organisms that do not have mitochondria, such as Entamoeba histolytica, Giardia intestinalis and several species of Microsporidia. These organisms are not capable of gaining energy from oxidative phosphorylation, which is normally performed by mitochondria.